{
  "gene_name": "Apoptosis-enhancing nuclease",
  "gene": "UniProtKB:Q8WTP8",
  "term_label": "intrinsic apoptotic signaling pathway in response to DNA damage by p53 class mediator",
  "term_id": "GO:0042771",
  "gene_symbol": "AEN"
}